{
  "gene": "UniProtKB:Q8TBZ6",
  "term_label": "nucleus",
  "term_id": "GO:0005634",
  "gene_symbol": "TRMT10A",
  "gene_name": "tRNA methyltransferase 10 homolog A"
}